{
  "gene": "UniProtKB:Q7Z6B0",
  "term_id": "GO:0090160",
  "gene_name": "Coiled-coil domain-containing protein 91",
  "gene_symbol": "CCDC91",
  "term_label": "Golgi to lysosome transport"
}